{
  "term_id": "GO:1905394",
  "gene_symbol": "WASHC2A",
  "gene_name": "WASH complex subunit 2A",
  "term_label": "retromer complex binding",
  "gene": "UniProtKB:Q641Q2"
}